cellular bud neck split septin rings [GO:0032177] (cellular component) Definition: Two separate septin rings that are formed from the septin collar at the time of cytokinesis in cells that divide by budding. These two rings are thought to delineate a special compartment in which factors involved in cytokinesis are concentrated. References: PMID:16009555 Sources: GOC:krc Relationships: is a type of cellular bud neck septin structure [GO:0000399]; is a type of GO:0032161; is a type of split septin rings [GO:0032176]